{
  "term_label": "alpha-mannosidase activity",
  "gene_name": "Alpha-mannosidase 2",
  "gene_symbol": "MAN2A1",
  "term_id": "GO:0004559",
  "gene": "UniProtKB:Q16706"
}